{
  "term_label": "positive regulation of canonical NF-kappaB signal transduction",
  "gene_symbol": "TRIM38",
  "gene": "UniProtKB:O00635",
  "gene_name": "E3 ubiquitin-protein ligase TRIM38",
  "term_id": "GO:0043123"
}